{
  "gene": "UniProtKB:Q16777",
  "gene_name": "Histone H2A type 2-C",
  "term_label": "heterochromatin formation",
  "gene_symbol": "H2AC20",
  "term_id": "GO:0031507"
}